{
  "gene": "UniProtKB:A8MWD9",
  "gene_symbol": "SNRPGP15",
  "term_label": "P granule",
  "gene_name": "Putative small nuclear ribonucleoprotein G-like protein 15",
  "term_id": "GO:0043186"
}